response to granulocyte macrophage colony-stimulating factor [GO:0097012] (biological process) Definition: Any process that results in a change in state or activity of a cell or an organism (in terms of movement, secretion, enzyme production, gene expression, etc.) as a result of a granulocyte macrophage colony-stimulating factor stimulus. Sources: GOC:pr Relationships: is a type of response to cytokine [GO:0034097] Subtypes: GO:0097011 Also known as: response to GM-CSF, response to granulocyte macrophage colony-stimulating factor stimulus